membrane lipid biosynthetic process [GO:0046467] (biological process) Also known as: membrane lipid anabolism, membrane lipid biosynthesis, membrane lipid formation, membrane lipid synthesis Definition: The chemical reactions and pathways resulting in the formation of membrane lipids, any lipid found in or associated with a biological membrane. Subtypes: glycolipid biosynthetic process [GO:0009247], GO:0030148 Relationships: is_a membrane lipid metabolic process [GO:0006643]; is a type of GO:0008610 Sources: GOC:ai